FMN binding [GO:0010181] (molecular function) Also known as: flavin mononucleotide binding Relationships: is a type of ribonucleotide binding [GO:0032553]; is a type of anion binding [GO:0043168] Definition: Binding to flavin mono nucleotide. Flavin mono nucleotide (FMN) is the coenzyme or the prosthetic group of various flavoprotein oxidoreductase enzymes. Sources: GOC:tb